{
  "term_label": "positive regulation of transcription by RNA polymerase II",
  "gene": "UniProtKB:P49116",
  "term_id": "GO:0045944",
  "gene_name": "Nuclear receptor subfamily 2 group C member 2",
  "gene_symbol": "NR2C2"
}